type II activin receptor binding [GO:0070699] (molecular function) Definition: Binding to a type II activin receptor. Sources: GOC:BHF, GOC:vk Relationships: is a type of activin receptor binding [GO:0070697]